{
  "gene_name": "ADP-ribosylation factor-like protein 8A",
  "gene_symbol": "ARL8A",
  "term_id": "GO:0005765",
  "gene": "UniProtKB:Q96BM9",
  "term_label": "lysosomal membrane"
}